negative regulation of flavonoid biosynthetic process [GO:0009964] (biological process) Sources: GOC:tb Relationships: is a type of negative regulation of biosynthetic process [GO:0009890]; is a type of GO:0009962; negatively regulates GO:0009813 Subtypes: negative regulation of anthocyanin biosynthetic process [GO:0031541], GO:1900385 Also known as: down regulation of flavonoid biosynthetic process, down-regulation of flavonoid biosynthetic process, downregulation of flavonoid biosynthetic process, negative regulation of flavonoid anabolism, negative regulation of flavonoid biosynthesis, negative regulation of flavonoid formation, negative regulation of flavonoid synthesis, inhibition of flavonoid biosynthetic process Definition: Any process that stops, prevents, or reduces the frequency, rate or extent of the chemical reactions and pathways resulting in the formation of flavonoids.